tRNA wobble uridine modification [GO:0002098] (biological process) Relationships: is_a tRNA wobble base modification [GO:0002097] Definition: The process in which a uridine at position 34 of a tRNA is post-transcriptionally modified. The wobble nucleoside of the tRNA sequence  (position 34) corresponds to the first position of the anticodon. Sources: GOC:hjd, ISBN:155581073X Subtypes: tRNA wobble position uridine thiolation [GO:0002143], tRNA wobble base 5-methoxycarbonylmethyl-2-thiouridinylation [GO:0002926], mitochondrial tRNA wobble uridine modification [GO:0070899]